{
  "term_id": "GO:0006218",
  "gene": "UniProtKB:O95045",
  "term_label": "uridine catabolic process",
  "gene_name": "Uridine phosphorylase 2",
  "gene_symbol": "UPP2"
}